cellular response to pulsatile fluid shear stress [GO:0097703] (biological process) Subtypes: GO:0097705 Definition: Any response to pulsatile fluid shear stress that occurs at the level of a cell. References: PMID:21768538 Sources: GOC:BHF, GOC:BHF_miRNA, GOC:bc Relationships: is a type of cellular response to fluid shear stress [GO:0071498]; is a type of GO:0097701